{
  "gene_name": "Mitochondrial import receptor subunit TOM34",
  "term_label": "cytosol",
  "term_id": "GO:0005829",
  "gene_symbol": "TOMM34",
  "gene": "UniProtKB:Q15785"
}